{
  "term_label": "Cul3-RING ubiquitin ligase complex",
  "term_id": "GO:0031463",
  "gene": "UniProtKB:Q53GT1",
  "gene_name": "Kelch-like protein 22",
  "gene_symbol": "KLHL22"
}